muscle adaptation [GO:0043500] (BP) Relationships: is a type of muscle system process [GO:0003012]; is a type of GO:0050896 References: PMID:11181628, PMID:11449884, PMID:12605307 Sources: GOC:mtg_muscle Subtypes: muscle hypertrophy in response to stress [GO:0003299], GO:0014805, GO:0014888, GO:0014889, GO:0014900 Also known as: muscle plasticity Definition: A process in which muscle adapts, with consequent modifications to structural and/or functional phenotypes, in response to a stimulus. Stimuli include contractile activity, loading conditions, substrate supply, and environmental factors. These adaptive events occur in both muscle fibers and associated structures (motoneurons and capillaries), and they involve alterations in regulatory mechanisms, contractile properties and metabolic capacities. Regulation: positively regulated by GO:0014744; negatively regulated by negative regulation of muscle adaptation [GO:0014745]; regulated by regulation of muscle adaptation [GO:0043502]